{
  "gene": "UniProtKB:O95685",
  "gene_name": "Protein phosphatase 1 regulatory subunit 3D",
  "gene_symbol": "PPP1R3D",
  "term_label": "regulation of glycogen biosynthetic process",
  "term_id": "GO:0005979"
}